lateral mesoderm development [GO:0048368] (BP) Also known as: lateral plate mesoderm development Sources: GOC:go_curators Relationships: is a type of GO:0007498; is_a GO:0060485 Definition: The process whose specific outcome is the progression of the lateral mesoderm over time, from its formation to the mature structure.